plasma membrane proton-transporting V-type ATPase, V1 domain [GO:0000223] (cellular component) Sources: GOC:mah Relationships: is a type of proton-transporting V-type ATPase, V1 domain [GO:0033180]; is a type of plasma membrane protein complex [GO:0098797]; is part of plasma membrane proton-transporting V-type ATPase complex [GO:0033181] Also known as: plasma membrane hydrogen ion-transporting ATPase V1 domain Definition: The V1 domain of a proton-transporting V-type ATPase found in the plasma membrane.